{
  "gene_symbol": "MMACHC",
  "gene": "UniProtKB:Q9Y4U1",
  "term_id": "GO:0009235",
  "gene_name": "Cyanocobalamin reductase _ alkylcobalamin dealkylase",
  "term_label": "cobalamin metabolic process"
}